{
  "gene": "UniProtKB:Q9UN36",
  "term_label": "signal transduction",
  "gene_symbol": "NDRG2",
  "gene_name": "Protein NDRG2",
  "term_id": "GO:0007165"
}